regulation of ascospore formation [GO:0034307] (biological process) Definition: Any process that modulates the frequency, rate or extent of ascospore formation. An example of this process is found in Saccharomyces cerevisiae. Sources: GOC:mah Also known as: MAPKKK cascade during sporulation Relationships: is a type of GO:0010564; is_a regulation of sexual sporulation resulting in formation of a cellular spore [GO:0043940]; is a type of regulation of cell development [GO:0060284]; regulates GO:0030437 Subtypes: positive regulation of ascospore formation [GO:0075296], negative regulation of ascospore formation [GO:0075297]